{
  "gene": "UniProtKB:Q8N436",
  "gene_symbol": "CPXM2",
  "term_label": "Unknown cellular component",
  "gene_name": "Inactive carboxypeptidase-like protein X2",
  "term_id": "UNKNOWN:0003"
}